{
  "term_label": "regulation of programmed cell death",
  "gene_name": "BCL2_adenovirus E1B 19 kDa protein-interacting protein 3-like",
  "term_id": "GO:0043067",
  "gene": "UniProtKB:O60238",
  "gene_symbol": "BNIP3L"
}